{
  "gene_name": "Dual specificity tyrosine-phosphorylation-regulated kinase 3",
  "gene_symbol": "DYRK3",
  "term_label": "positive regulation of cell cycle G2/M phase transition",
  "gene": "UniProtKB:O43781",
  "term_id": "GO:1902751"
}